{
  "gene_symbol": "ZC3H15",
  "gene_name": "Zinc finger CCCH domain-containing protein 15",
  "gene": "UniProtKB:Q8WU90",
  "term_label": "Unknown molecular function",
  "term_id": "UNKNOWN:0001"
}